glomerular mesangium development [GO:0072109] (biological process) Definition: The process whose specific outcome is the progression of the glomerular mesangium over time, from its formation to the mature structure. The glomerular mesangium is the thin membrane connective tissue composed of mesangial cells, which helps to support the capillary loops in a renal glomerulus. Sources: GOC:mtg_kidney_jan10 Relationships: is a type of GO:0061448; BFO_0000050 glomerulus vasculature development [GO:0072012] Subtypes: mesonephric glomerular mesangium development [GO:0061247], GO:0072223